{
  "term_label": "Unknown molecular function",
  "gene_name": "Centrosomal protein of 112 kDa",
  "gene": "UniProtKB:Q8N8E3",
  "gene_symbol": "CEP112",
  "term_id": "UNKNOWN:0001"
}